{
  "gene": "UniProtKB:P31270",
  "term_id": "GO:0060272",
  "term_label": "embryonic skeletal joint morphogenesis",
  "gene_name": "Homeobox protein Hox-A11",
  "gene_symbol": "HOXA11"
}